{
  "term_label": "tRNA binding",
  "gene_symbol": "PTCD1",
  "gene_name": "Pentatricopeptide repeat-containing protein 1, mitochondrial",
  "gene": "UniProtKB:O75127",
  "term_id": "GO:0000049"
}